regulation of stomach neuroendocrine cell differentiation [GO:0061105] (biological process) Subtypes: negative regulation of stomach neuroendocrine cell differentiation [GO:0061106] Definition: Any process that modulates the rate, frequency or extent of the differentiation of a neuroendocrine cell in the stomach. Sources: GOC:dph Relationships: is a type of GO:0030856; is a type of regulation of neuron differentiation [GO:0045664]; regulates stomach neuroendocrine cell differentiation [GO:0061102]